{
  "term_label": "nucleus",
  "term_id": "GO:0005634",
  "gene_symbol": "RBMS3",
  "gene_name": "RNA-binding motif, single-stranded-interacting protein 3",
  "gene": "UniProtKB:Q6XE24"
}